{
  "term_label": "cytokine binding",
  "term_id": "GO:0019955",
  "gene_name": "Growth hormone receptor",
  "gene": "UniProtKB:P10912",
  "gene_symbol": "GHR"
}